{
  "gene": "UniProtKB:Q96NG8",
  "gene_name": "Zinc finger protein 582",
  "term_id": "GO:0000981",
  "gene_symbol": "ZNF582",
  "term_label": "DNA-binding transcription factor activity, RNA polymerase II-specific"
}